adult visceral muscle development [GO:0007524] (biological process) Definition: The process whose specific outcome is the progression of the adult visceral muscle over time, from its formation to the mature structure. Relationships: is a type of visceral muscle development [GO:0007522] Sources: GOC:jid